{
  "gene": "UniProtKB:Q6ZS62",
  "gene_symbol": "COLCA1",
  "gene_name": "Colorectal cancer-associated protein 1",
  "term_label": "Unknown molecular function",
  "term_id": "UNKNOWN:0001"
}